{
  "gene_name": "ATP-dependent 6-phosphofructokinase, liver type",
  "gene": "UniProtKB:P17858",
  "term_label": "fructose 1,6-bisphosphate metabolic process",
  "term_id": "GO:0030388",
  "gene_symbol": "PFKL"
}